{
  "gene_symbol": "ATP5MC3",
  "term_label": "Unknown molecular function",
  "term_id": "UNKNOWN:0001",
  "gene": "UniProtKB:P48201",
  "gene_name": "ATP synthase F(0) complex subunit C3, mitochondrial"
}